ajugose biosynthetic process using galactan:galactan galactosyltransferase [GO:0033538] (biological process) Definition: The chemical reactions and pathways resulting in the formation of ajugose, the hexasaccharide beta-D-fructofuranosyl alpha-D-galactopyranosyl-(1->6)-alpha-D-galactopyranosyl-(1->6)-alpha-D-galactopyranosyl-(1->6)-alpha-D-galactopyranosyl-(1->6)-alpha-D-glucopyranoside, by a pathway in which galactan:galactan galactosyltransferase catalyzes chain elongation by transferring the alpha-galactosyl residue of one raffinose-family oligosaccharide to another. Relationships: is a type of GO:0033536 Also known as: ajugose anabolism using galactan:galactan galactosyltransferase, ajugose biosynthesis using galactan:galactan galactosyltransferase, ajugose formation using galactan:galactan galactosyltransferase, ajugose synthesis using galactan:galactan galactosyltransferase Sources: GOC:mah, MetaCyc:PWY-5343